{
  "term_label": "glucuronosyltransferase activity",
  "gene_symbol": "UGT3A2",
  "term_id": "GO:0015020",
  "gene": "UniProtKB:Q3SY77",
  "gene_name": "UDP-glucuronosyltransferase 3A2"
}